{
  "gene_symbol": "MACF1",
  "gene": "UniProtKB:Q9UPN3",
  "gene_name": "Microtubule-actin cross-linking factor 1, isoforms 1_2_3_4_5",
  "term_id": "GO:0005874",
  "term_label": "microtubule"
}